{
  "gene": "UniProtKB:Q9H903",
  "term_label": "methylenetetrahydrofolate dehydrogenase (NADP+) activity",
  "term_id": "GO:0004488",
  "gene_symbol": "MTHFD2L",
  "gene_name": "Bifunctional methylenetetrahydrofolate dehydrogenase_cyclohydrolase 2, mitochondrial"
}